regulation of transcription from RNA polymerase II promoter by glucose [GO:0000430] (BP) Relationships: is a type of carbon catabolite regulation of transcription from RNA polymerase II promoter [GO:0000429]; is a type of regulation of transcription by glucose [GO:0046015] Sources: GOC:krc Definition: Any process involving glucose that modulates the frequency, rate or extent of transcription from an RNA polymerase II promoter. Subtypes: positive regulation of transcription from RNA polymerase II promoter by glucose [GO:0000432], GO:0061987